{
  "term_id": "UNKNOWN:0001",
  "gene": "UniProtKB:Q6ZU80",
  "term_label": "Unknown molecular function",
  "gene_name": "Centrosomal protein of 128 kDa",
  "gene_symbol": "CEP128"
}